{
  "gene_symbol": "LAMTOR1",
  "gene": "UniProtKB:Q6IAA8",
  "term_id": "GO:0005765",
  "term_label": "lysosomal membrane",
  "gene_name": "Ragulator complex protein LAMTOR1"
}